{
  "gene": "UniProtKB:Q13813",
  "gene_symbol": "SPTAN1",
  "gene_name": "Spectrin alpha chain, non-erythrocytic 1",
  "term_id": "GO:0030054",
  "term_label": "cell junction"
}